D-galactonate transmembrane transporter activity [GO:0042881] (molecular function) Sources: GOC:jl, GOC:jsg, GOC:mah, GOC:mtg_transport, ISBN:0198506732 Definition: Enables the transfer of D-galactonate, the D-enantiomer of galactonate, from one side of a membrane to the other. Relationships: is a type of monocarboxylic acid transmembrane transporter activity [GO:0008028]; is a type of carbohydrate transmembrane transporter activity [GO:0015144]; is a type of GO:0042879; is part of D-galactonate transmembrane transport [GO:0042875]